{
  "term_label": "positive regulation of synaptic transmission",
  "gene_name": "Calsyntenin-1",
  "term_id": "GO:0050806",
  "gene": "UniProtKB:O94985",
  "gene_symbol": "CLSTN1"
}